regulation of sporangium germination [GO:0075223] (biological process) Subtypes: positive regulation of sporangium germination [GO:0075224], negative regulation of sporangium germination [GO:0075225] Definition: Any process that modulates the frequency, rate or extent of sporangium germination. Sources: GOC:pamgo_curators Relationships: is a type of regulation of sporangium development [GO:0075310]; regulates GO:0075222 Also known as: modulation of sporangium germination, modulation of sporangium germination on or near host